2-formylbenzoate dehydrogenase (NAD+) activity [GO:0018474] (molecular function) Relationships: is a type of GO:0004029 Definition: Catalysis of the reaction: 2-formylbenzoate + H2O + NAD+ = 2 H+ + NADH + phthalate. Sources: RHEA:27298 Also known as: 2-carboxybenzaldehyde dehydrogenase activity